{
  "term_id": "GO:0003700",
  "gene_symbol": "ZNF212",
  "gene": "UniProtKB:Q9UDV6",
  "gene_name": "Zinc finger protein 212",
  "term_label": "DNA-binding transcription factor activity"
}